{
  "gene": "UniProtKB:A0PK05",
  "term_label": "Unknown molecular function",
  "gene_name": "Transmembrane protein 72",
  "term_id": "UNKNOWN:0001",
  "gene_symbol": "TMEM72"
}